glutathionylspermidine synthase activity [GO:0008885] (molecular function) Definition: Catalysis of the reaction: gamma-L-glutamyl-L-cysteinyl-glycine + spermidine + ATP = N1-(gamma-L-glutamyl-L-cysteinyl-glycyl)-spermidine + ADP + phosphate. Sources: EC:6.3.1.8 Also known as: GSP synthetase activity, gamma-L-glutamyl-L-cysteinyl-glycine:spermidine ligase (ADP-forming) [spermidine is numbered so that atom N-1 is in the amino group of the aminopropyl part of the molecule], gamma-L-glutamyl-L-cysteinyl-glycine:spermidine ligase (ADP-forming) activity, glutathione:spermidine ligase (ADP-forming) activity, glutathionylspermidine synthetase activity Relationships: is a type of GO:0016880